{
  "term_label": "natural killer cell lectin-like receptor binding",
  "gene_name": "UL16-binding protein 6",
  "term_id": "GO:0046703",
  "gene_symbol": "RAET1L",
  "gene": "UniProtKB:Q5VY80"
}